{
  "term_id": "GO:0095500",
  "gene_symbol": "LY6S",
  "gene": "UniProtKB:P0DTL4",
  "gene_name": "Lymphocyte antigen 6S",
  "term_label": "acetylcholine receptor signaling pathway"
}